xylan endo-1,3-beta-xylosidase activity [GO:0033905] (molecular function) Definition: Catalysis of the random hydrolysis of (1->3)-beta-D-glycosidic linkages in (1->3)-beta-D-xylans. Sources: EC:3.2.1.32 Also known as: xylanase activity, 1,3-beta-D-xylan xylanohydrolase activity, 1,3-beta-xylanase activity, 1,3-xylanase activity, beta-1,3-xylanase activity, endo-1,3-beta-xylanase activity, endo-1,3-xylanase activity, endo-beta-1,3-xylanase activity Relationships: is a type of xylanase activity [GO:0097599]